{
  "term_id": "GO:0005543",
  "gene_symbol": "GLE1",
  "gene": "UniProtKB:Q53GS7",
  "term_label": "phospholipid binding",
  "gene_name": "mRNA export factor GLE1"
}